{
  "gene_name": "E3 ubiquitin-protein ligase Jade-2",
  "gene_symbol": "JADE2",
  "term_id": "GO:0005634",
  "gene": "UniProtKB:Q9NQC1",
  "term_label": "nucleus"
}